regulation of FACT complex assembly [GO:1905644] (biological process) Definition: Any process that modulates the frequency, rate or extent of FACT complex assembly. Relationships: is a type of GO:0043254; regulates FACT complex assembly [GO:1905635] Also known as: regulation of FACT complex formation, regulation of Facilitates chromatin transcription complex assembly, regulation of Facilitates chromatin transcription complex formation References: PMID:20889714 Sources: GOC:TermGenie, GO_REF:0000058 Subtypes: GO:1905645, positive regulation of FACT complex assembly [GO:1905646]